{
  "gene_symbol": "PCTP",
  "gene": "UniProtKB:Q9UKL6",
  "term_label": "Unknown biological process",
  "gene_name": "Phosphatidylcholine transfer protein",
  "term_id": "UNKNOWN:0002"
}